{
  "term_id": "GO:0050113",
  "gene_name": "Inositol oxygenase",
  "gene": "UniProtKB:Q9UGB7",
  "term_label": "inositol oxygenase activity",
  "gene_symbol": "MIOX"
}